{
  "term_label": "cellular response to exogenous dsRNA",
  "term_id": "GO:0071360",
  "gene": "UniProtKB:Q8N884",
  "gene_symbol": "CGAS",
  "gene_name": "Cyclic GMP-AMP synthase"
}